glycolate oxidase complex [GO:0009339] (cellular component) Relationships: is a type of oxidoreductase complex [GO:1990204]; is part of cytoplasm [GO:0005737] References: PMID:4557653, PMID:8606183 Definition: An enzyme complex that catalyzes the oxidation of 2-hydroxy acid to form 2-oxo acid and hydrogen peroxide (H2O2). The enzyme is a flavoprotein (FMN).